{
  "gene": "UniProtKB:P05109",
  "gene_name": "Protein S100-A8",
  "term_label": "neutrophil chemotaxis",
  "gene_symbol": "S100A8",
  "term_id": "GO:0030593"
}